{
  "term_id": "GO:0003954",
  "gene_symbol": "ENOX1",
  "term_label": "NADH dehydrogenase activity",
  "gene": "UniProtKB:Q8TC92",
  "gene_name": "Ecto-NOX disulfide-thiol exchanger 1"
}